{
  "gene_symbol": "TRIOBP",
  "gene": "UniProtKB:Q9H2D6",
  "term_id": "GO:0015629",
  "gene_name": "TRIO and F-actin-binding protein",
  "term_label": "actin cytoskeleton"
}